TORC2 complex binding [GO:1904841] (molecular function) Note: Binding to a TORC2 complex, a protein complex that mediates the phosphorylation of protein kinase B Definition: Binding to a TORC2 complex. Also known as: TOR complex 2 binding, TORC 2 complex binding, TORC2 binding, rapamycin and nutrient-insensitive TOR complex binding, mTORC2 binding Relationships: is a type of protein-containing complex binding [GO:0044877] References: PMID:20660630 Sources: GOC:TermGenie